{
  "gene_name": "Carbohydrate sulfotransferase 9",
  "gene_symbol": "CHST9",
  "term_label": "sulfotransferase activity",
  "gene": "UniProtKB:Q7L1S5",
  "term_id": "GO:0008146"
}